{
  "gene_name": "Peroxisomal carnitine O-octanoyltransferase",
  "term_id": "UNKNOWN:0002",
  "gene_symbol": "CROT",
  "term_label": "Unknown biological process",
  "gene": "UniProtKB:Q9UKG9"
}